{
  "term_id": "GO:0006869",
  "gene_name": "ATP-binding cassette sub-family A member 9",
  "gene_symbol": "ABCA9",
  "term_label": "lipid transport",
  "gene": "UniProtKB:Q8IUA7"
}